{
  "term_id": "UNKNOWN:0001",
  "gene": "UniProtKB:Q96A19",
  "term_label": "Unknown molecular function",
  "gene_name": "Coiled-coil domain-containing protein 102A",
  "gene_symbol": "CCDC102A"
}